{
  "gene": "UniProtKB:Q6ZQT0",
  "gene_name": "Putative uncharacterized protein FLJ45035",
  "term_id": "UNKNOWN:0001",
  "gene_symbol": "Q6ZQT0",
  "term_label": "Unknown molecular function"
}